{
  "gene": "UniProtKB:O95229",
  "term_id": "GO:0016604",
  "gene_symbol": "ZWINT",
  "gene_name": "ZW10 interactor",
  "term_label": "nuclear body"
}